salt transmembrane transporter activity [GO:1901702] (molecular function) Definition: Enables the transfer of salt from one side of a membrane to the other. Relationships: is_a transmembrane transporter activity [GO:0022857] Sources: GOC:TermGenie, GOC:pr Subtypes: GO:0015143, tartrate transmembrane transporter activity [GO:0015554]